positive regulation of mitochondrial membrane permeability [GO:0035794] (BP) References: PMID:12546810 Sources: GOC:bf Definition: Any process that increases the frequency, rate or extent of the passage or uptake of molecules by the mitochondrial membrane. Relationships: is a type of regulation of mitochondrial membrane permeability [GO:0046902]; is a type of positive regulation of membrane permeability [GO:1905710] Subtypes: positive regulation of mitochondrial outer membrane permeabilization involved in apoptotic signaling pathway [GO:1901030], mitochondrial outer membrane permeabilization involved in programmed cell death [GO:1902686] Also known as: positive regulation of transport across mitochondrial membrane, MPT, mitochondrial membrane permeability transition, mitochondrial membrane permeabilization, mitochondrial permeability transition